{
  "gene": "UniProtKB:Q8N6C8",
  "gene_symbol": "LILRA3",
  "term_label": "immune response-inhibiting cell surface receptor signaling pathway",
  "gene_name": "Leukocyte immunoglobulin-like receptor subfamily A member 3",
  "term_id": "GO:0002767"
}